{
  "gene_name": "KH domain-containing protein 3",
  "term_id": "GO:0032991",
  "gene": "UniProtKB:Q587J8",
  "gene_symbol": "KHDC3L",
  "term_label": "protein-containing complex"
}